{
  "gene_name": "Collagen alpha-1(XXIII) chain",
  "term_id": "GO:0030198",
  "term_label": "extracellular matrix organization",
  "gene_symbol": "COL23A1",
  "gene": "UniProtKB:Q86Y22"
}